regulation of endocytic recycling [GO:2001135] (biological process) Also known as: regulation of retrograde transport of endocytic vesicles Definition: Any process that modulates the frequency, rate or extent of endocytic recycling. Sources: GOC:obol Subtypes: regulation of endosome to plasma membrane protein transport [GO:1905749], negative regulation of endocytic recycling [GO:2001136], positive regulation of endocytic recycling [GO:2001137] Relationships: is a type of regulation of intracellular transport [GO:0032386]; is a type of regulation of vesicle-mediated transport [GO:0060627]; regulates GO:0032456